{
  "term_id": "GO:0000463",
  "gene_symbol": "PAK1IP1",
  "gene_name": "p21-activated protein kinase-interacting protein 1",
  "term_label": "maturation of LSU-rRNA from tricistronic rRNA transcript (SSU-rRNA, 5.8S rRNA, LSU-rRNA)",
  "gene": "UniProtKB:Q9NWT1"
}